septin cytoskeleton [GO:0032156] (cellular component) Definition: The part of the cytoskeleton (the internal framework of a cell) composed of septins and associated proteins. Includes septin cytoskeleton-associated complexes. Sources: GOC:mah Relationships: is a type of cytoskeleton [GO:0005856] Subtypes: septin ring [GO:0005940], septin cap [GO:0032159], GO:0032160, septin collar [GO:0032173], split septin rings [GO:0032176], postsynaptic septin cytoskeleton [GO:0150050]